alanine catabolic process [GO:0006524] (biological process) Subtypes: L-alanine catabolic process [GO:0042853], D-alanine catabolic process [GO:0055130] Relationships: is_a GO:0006522; is a type of alpha-amino acid catabolic process [GO:1901606] Sources: GOC:go_curators Definition: The chemical reactions and pathways resulting in the breakdown of alanine, 2-aminopropanoic acid. Also known as: alanine breakdown, alanine catabolism, alanine degradation